{
  "term_label": "negative regulation of DNA-templated transcription",
  "gene_symbol": "CBFA2T2",
  "term_id": "GO:0045892",
  "gene": "UniProtKB:O43439",
  "gene_name": "Protein CBFA2T2"
}